{
  "gene_name": "Histone H2B type 1-B",
  "gene_symbol": "H2BC3",
  "term_id": "GO:0000786",
  "term_label": "nucleosome",
  "gene": "UniProtKB:P33778"
}